{
  "term_label": "autophagosome assembly",
  "term_id": "GO:0000045",
  "gene_symbol": "GABARAPL3",
  "gene": "UniProtKB:Q9BY60",
  "gene_name": "Gamma-aminobutyric acid receptor-associated protein-like 3"
}